{
  "term_id": "UNKNOWN:0002",
  "gene_symbol": "DNPEP",
  "term_label": "Unknown biological process",
  "gene": "UniProtKB:Q9ULA0",
  "gene_name": "Aspartyl aminopeptidase"
}